{
  "gene_name": "ATP-dependent RNA helicase DHX29",
  "gene_symbol": "DHX29",
  "gene": "UniProtKB:Q7Z478",
  "term_label": "RNA binding",
  "term_id": "GO:0003723"
}